{
  "term_id": "GO:0006112",
  "term_label": "energy reserve metabolic process",
  "gene_name": "Leptin",
  "gene": "UniProtKB:P41159",
  "gene_symbol": "LEP"
}